{
  "gene_name": "RNA N6-adenosine-methyltransferase METTL16",
  "gene_symbol": "METTL16",
  "term_id": "GO:0005634",
  "gene": "UniProtKB:Q86W50",
  "term_label": "nucleus"
}